{
  "gene_symbol": "TRIL",
  "term_label": "plasma membrane",
  "gene": "UniProtKB:Q7L0X0",
  "gene_name": "TLR4 interactor with leucine rich repeats",
  "term_id": "GO:0005886"
}